lipoprotein lipase activator activity [GO:0060230] (molecular function) References: PMID:10727238 Sources: GOC:BHF, GOC:dph, GOC:tb Relationships: is a type of lipase activator activity [GO:0060229]; positively regulates lipoprotein lipase activity [GO:0004465] Definition: Binds to and increases the activity of a lipoprotein lipase, an enzyme that catalyzes of the hydrolysis of a lipid within a lipoprotein.